{
  "term_label": "Unknown cellular component",
  "term_id": "UNKNOWN:0003",
  "gene_symbol": "LGALSL",
  "gene_name": "Galectin-related protein",
  "gene": "UniProtKB:Q3ZCW2"
}